{
  "term_label": "chromatin organization",
  "gene_name": "Putative Dresden prostate carcinoma protein 2",
  "gene": "UniProtKB:Q86SG4",
  "gene_symbol": "HMGN2P46",
  "term_id": "GO:0006325"
}